{
  "gene_name": "CTP synthase 2",
  "gene_symbol": "CTPS2",
  "term_label": "cytoophidium",
  "gene": "UniProtKB:Q9NRF8",
  "term_id": "GO:0097268"
}